ventricular cardiac muscle tissue morphogenesis [GO:0055010] (biological process) Definition: The process in which the anatomical structures of cardiac ventricle muscle is generated and organized. Sources: GOC:devbiol Relationships: is_a cardiac muscle tissue morphogenesis [GO:0055008]; is part of GO:0003208; is part of ventricular cardiac muscle tissue development [GO:0003229] Also known as: cardiac ventricle muscle morphogenesis, ventricular heart muscle morphogenesis Subtypes: left ventricular cardiac muscle tissue morphogenesis [GO:0003220], right ventricular cardiac muscle tissue morphogenesis [GO:0003221], ventricular trabecula myocardium morphogenesis [GO:0003222], ventricular compact myocardium morphogenesis [GO:0003223]